mRNA 5'-UTR binding [GO:0048027] (molecular function) Relationships: is a type of mRNA binding [GO:0003729] Sources: GOC:jid Definition: Binding to an mRNA molecule at its 5' untranslated region. Also known as: mRNA 5' UTR binding